{
  "term_id": "GO:0016020",
  "term_label": "membrane",
  "gene": "UniProtKB:P30954",
  "gene_symbol": "OR10J1",
  "gene_name": "Olfactory receptor 10J1"
}